double-strand break repair via nonhomologous end joining [GO:0006303] (biological process) Regulation: regulated by GO:2001032; negatively regulated by negative regulation of double-strand break repair via nonhomologous end joining [GO:2001033]; positively regulated by positive regulation of double-strand break repair via nonhomologous end joining [GO:2001034] Relationships: is a type of double-strand break repair [GO:0006302] References: PMID:10827453, PMID:24837021 Sources: GOC:rph Subtypes: double-strand break repair via classical nonhomologous end joining [GO:0097680], double-strand break repair via alternative nonhomologous end joining [GO:0097681] Definition: The repair of a double-strand break in DNA in which the two broken ends are rejoined with little or no sequence complementarity. Information at the DNA ends may be lost due to the modification of broken DNA ends. This term covers instances of separate pathways, called classical (or canonical) and alternative nonhomologous end joining (C-NHEJ and A-NHEJ). These in turn may further branch into sub-pathways, but evidence is still unclear. Also known as: NHEJ